{
  "gene_name": "Fas-activated serine_threonine kinase",
  "gene_symbol": "FASTK",
  "gene": "UniProtKB:Q14296",
  "term_label": "regulation of mitochondrial mRNA stability",
  "term_id": "GO:0044528"
}